{
  "gene_name": "Metal cation symporter ZIP14",
  "term_label": "zinc ion transmembrane transporter activity",
  "gene": "UniProtKB:Q15043",
  "term_id": "GO:0005385",
  "gene_symbol": "SLC39A14"
}